{
  "term_label": "immunoglobulin complex",
  "term_id": "GO:0019814",
  "gene": "UniProtKB:A0A0C4DH90",
  "gene_symbol": "IGKV3OR2-268",
  "gene_name": "Immunoglobulin kappa variable 3_OR2-268 (non-functional) (Fragment)"
}